positive regulation of prolactin secretion [GO:1902722] (biological process) References: PMID:16159377 Sources: GOC:TermGenie, GO_REF:0000058 Relationships: is a type of positive regulation of protein secretion [GO:0050714]; is a type of positive regulation of peptide hormone secretion [GO:0090277]; positively regulates GO:0070459 Also known as: up regulation of prolactin secretion, up-regulation of prolactin secretion, upregulation of prolactin secretion, activation of prolactin secretion Definition: Any process that activates or increases the frequency, rate or extent of prolactin secretion.